{
  "term_id": "GO:0008528",
  "gene": "UniProtKB:P34998",
  "gene_symbol": "CRHR1",
  "term_label": "G protein-coupled peptide receptor activity",
  "gene_name": "Corticotropin-releasing factor receptor 1"
}